{
  "term_label": "cell differentiation",
  "term_id": "GO:0030154",
  "gene_symbol": "RXRG",
  "gene_name": "Retinoic acid receptor RXR-gamma",
  "gene": "UniProtKB:P48443"
}